{
  "gene": "UniProtKB:Q5TC84",
  "gene_symbol": "OGFRL1",
  "term_label": "Unknown cellular component",
  "term_id": "UNKNOWN:0003",
  "gene_name": "Opioid growth factor receptor-like protein 1"
}